{
  "gene": "UniProtKB:Q9HBG6",
  "gene_symbol": "IFT122",
  "term_label": "intraciliary retrograde transport",
  "gene_name": "Intraflagellar transport protein 122 homolog",
  "term_id": "GO:0035721"
}